pICln-Sm protein complex [GO:0034715] (cellular component) Also known as: 6S pICln complex Relationships: is a type of Sm-like protein family complex [GO:0120114]; is part of cytoplasm [GO:0005737] References: PMID:11713266 Sources: GOC:mah Definition: A protein complex that contains pICln (CLNS1A) and several Sm proteins, including SmD1, SmD2, SmE, SmF, and SmG.